{
  "gene": "UniProtKB:Q96P68",
  "gene_name": "2-oxoglutarate receptor 1",
  "gene_symbol": "OXGR1",
  "term_label": "signaling receptor activity",
  "term_id": "GO:0038023"
}